U6 snRNA (adenine-(43)-N(6))-methyltransferase activity [GO:0120048] (molecular function) References: PMID:28525753, PMID:32266935 Sources: RHEA:52808 Definition: Catalysis of the reaction: adenosine in U6 snRNA + S-adenosyl-L-methionine = H+ + N(6)-methyladenosine in U6 snRNA + S-adenosyl-L-homocysteine. Relationships: is a type of GO:0106346